{
  "term_label": "calcium ion binding",
  "gene_name": "Fer-1-like protein 5",
  "gene": "UniProtKB:A0AVI2",
  "gene_symbol": "FER1L5",
  "term_id": "GO:0005509"
}